{
  "term_id": "GO:0010997",
  "gene": "UniProtKB:Q9UM11",
  "gene_symbol": "FZR1",
  "gene_name": "Fizzy-related protein homolog",
  "term_label": "anaphase-promoting complex binding"
}